{
  "gene": "UniProtKB:P20073",
  "gene_name": "Annexin A7",
  "term_label": "nucleus",
  "term_id": "GO:0005634",
  "gene_symbol": "ANXA7"
}